{
  "term_id": "GO:0005789",
  "gene": "UniProtKB:Q13724",
  "term_label": "endoplasmic reticulum membrane",
  "gene_name": "Mannosyl-oligosaccharide glucosidase",
  "gene_symbol": "MOGS"
}